{
  "gene": "UniProtKB:Q86Z23",
  "term_label": "synapse",
  "term_id": "GO:0045202",
  "gene_name": "Complement C1q-like protein 4",
  "gene_symbol": "C1QL4"
}